peptidyl-glutamine modification [GO:0018199] (BP) Definition: The modification of peptidyl-glutamine. Relationships: is_a peptidyl-amino acid modification [GO:0018193] Sources: GOC:go_curators Subtypes: peptidyl-pyroglutamic acid biosynthetic process, using glutaminyl-peptide cyclotransferase [GO:0017186], N-terminal peptidyl-glutamine acetylation [GO:0017192], isopeptide cross-linking via N6-(L-isoglutamyl)-L-lysine [GO:0018153]